{
  "term_id": "GO:0045943",
  "gene": "UniProtKB:P0CB47",
  "gene_symbol": "UBTFL1",
  "gene_name": "Upstream-binding factor 1-like protein 1",
  "term_label": "positive regulation of transcription by RNA polymerase I"
}